{
  "gene_name": "Golgin subfamily A member 7",
  "gene_symbol": "GOLGA7",
  "gene": "UniProtKB:Q7Z5G4",
  "term_label": "Unknown molecular function",
  "term_id": "UNKNOWN:0001"
}